{
  "gene_name": "Putative uncharacterized protein C3orf49",
  "gene": "UniProtKB:Q96BT1",
  "term_label": "Unknown cellular component",
  "gene_symbol": "C3orf49",
  "term_id": "UNKNOWN:0003"
}